alpha-glucoside transmembrane transporter activity [GO:0015151] (MF) References: PMID:28510148 Sources: GOC:jl, GOC:mtg_transport, ISBN:0198506732, ISBN:0815340729 Definition: Enables the transfer of alpha-glucosides from one side of a membrane to the other. Alpha-glucosides are glycosides in which the sugar group is a glucose residue, and the anomeric carbon of the bond is in an alpha configuration. Relationships: is a type of glucoside transmembrane transporter activity [GO:0042947]; is part of alpha-glucoside transport [GO:0000017] Subtypes: GO:0005352